{
  "gene": "UniProtKB:Q5XX13",
  "term_id": "UNKNOWN:0003",
  "gene_name": "F-box_WD repeat-containing protein 10",
  "term_label": "Unknown cellular component",
  "gene_symbol": "FBXW10"
}